nuclear SCF ubiquitin ligase complex [GO:0043224] (cellular component) Also known as: nuclear SCF complex, nuclear Skp1/Cul1/F-box protein complex, nuclear cullin complex References: PMID:15571813, PMID:15688063 Relationships: is a type of nuclear ubiquitin ligase complex [GO:0000152]; is a type of GO:0019005 Definition: A ubiquitin ligase complex, located in the nucleus, in which a cullin from the Cul1 subfamily and a RING domain protein form the catalytic core; substrate specificity is conferred by a Skp1 adaptor and an F-box protein. SCF complexes are involved in targeting proteins for degradation by the proteasome. The best characterized complexes are those from yeast and mammals (with core subunits named Cdc53/Cul1, Rbx1/Hrt1/Roc1).